{
  "gene_name": "mRNA turnover protein 4 homolog",
  "gene": "UniProtKB:Q9UKD2",
  "term_label": "rRNA processing",
  "term_id": "GO:0006364",
  "gene_symbol": "MRTO4"
}